{
  "gene": "UniProtKB:Q96JD6",
  "gene_name": "1,5-anhydro-D-fructose reductase",
  "term_label": "aldose reductase (NADPH) activity",
  "gene_symbol": "AKR1E2",
  "term_id": "GO:0004032"
}